{
  "gene_symbol": "TMEM40",
  "term_id": "UNKNOWN:0001",
  "gene": "UniProtKB:Q8WWA1",
  "gene_name": "Transmembrane protein 40",
  "term_label": "Unknown molecular function"
}